{
  "term_label": "nucleus",
  "gene_name": "Ubiquitin-conjugating enzyme E2 variant 1",
  "gene": "UniProtKB:Q13404",
  "term_id": "GO:0005634",
  "gene_symbol": "UBE2V1"
}